positive regulation of hypoxia-inducible factor-1alpha signaling pathway [GO:1902073] (BP) Definition: Any process that activates or increases the frequency, rate or extent of hypoxia-inducible factor-1alpha signaling pathway. References: PMID:21685248 Sources: GOC:TermGenie, GOC:bf Relationships: is a type of GO:1902071; is a type of GO:1902533; positively regulates hypoxia-inducible factor-1alpha signaling pathway [GO:0097411] Also known as: activation of HIF1alpha pathway, activation of hypoxia-inducible factor-1alpha signalling pathway, positive regulation of HIF1alpha pathway, positive regulation of hypoxia-inducible factor-1alpha signalling pathway, up regulation of HIF1alpha pathway, up regulation of hypoxia-inducible factor-1alpha signaling pathway, up regulation of hypoxia-inducible factor-1alpha signalling pathway, up-regulation of HIF1alpha pathway, up-regulation of hypoxia-inducible factor-1alpha signaling pathway, up-regulation of hypoxia-inducible factor-1alpha signalling pathway, upregulation of HIF1alpha pathway, upregulation of hypoxia-inducible factor-1alpha signaling pathway, upregulation of hypoxia-inducible factor-1alpha signalling pathway, activation of hypoxia-inducible factor-1alpha signaling pathway, hypoxic stabilization of HIF1A